{
  "gene_name": "Vascular endothelial growth factor receptor 1",
  "term_id": "GO:0005886",
  "term_label": "plasma membrane",
  "gene_symbol": "FLT1",
  "gene": "UniProtKB:P17948"
}